{
  "gene_symbol": "PABPC1L2A",
  "term_id": "GO:0008143",
  "gene": "UniProtKB:Q5JQF8",
  "gene_name": "Polyadenylate-binding protein 1-like 2",
  "term_label": "poly(A) binding"
}